axial mesoderm formation [GO:0048320] (biological process) Sources: GOC:dgh Relationships: is a type of GO:0001707; is part of GO:0048319 Definition: The process that gives rise to the axial mesoderm. This process pertains to the initial formation of the structure from unspecified parts.